{
  "gene_symbol": "USP17L23",
  "gene": "UniProtKB:D6RBM5",
  "gene_name": "Putative ubiquitin carboxyl-terminal hydrolase 17-like protein 23",
  "term_label": "Unknown molecular function",
  "term_id": "UNKNOWN:0001"
}